5'-3' DNA helicase activity [GO:0043139] (molecular function) Relationships: is a type of DNA helicase activity [GO:0003678] Sources: EC:5.6.2.3, GOC:jl Also known as: 5' to 3' DNA helicase activity, ATP-dependent 5' to 3' DNA helicase activity, ATP-dependent 5'-3' DNA helicase activity, DNA helicase IV activity Definition: Unwinding a DNA helix in the 5' to 3' direction, driven by ATP hydrolysis.